{
  "gene_name": "DNA repair protein complementing XP-A cells",
  "gene_symbol": "XPA",
  "term_id": "GO:0000110",
  "term_label": "nucleotide-excision repair factor 1 complex",
  "gene": "UniProtKB:P23025"
}